IMP catabolic process [GO:0006204] (biological process) Definition: The chemical reactions and pathways resulting in the breakdown of IMP, inosine monophosphate. Also known as: IMP breakdown, IMP catabolism, IMP degradation Relationships: is a type of purine ribonucleotide catabolic process [GO:0009154]; is a type of purine ribonucleoside monophosphate catabolic process [GO:0009169]; is a type of IMP metabolic process [GO:0046040] Sources: ISBN:0198506732